{
  "gene_symbol": "IFT56",
  "term_id": "GO:0097546",
  "gene": "UniProtKB:A0AVF1",
  "gene_name": "Intraflagellar transport protein 56",
  "term_label": "ciliary base"
}